negative regulation of cytosolic calcium ion concentration [GO:0051481] (biological process) Relationships: is_a regulation of biological quality [GO:0065008] Also known as: cytoplasmic calcium ion concentration reduction, reduction of calcium ion concentration in cytoplasm, reduction of cytoplasmic calcium ion concentration, cytosolic calcium ion concentration reduction, reduction of calcium ion concentration in cytosol, reduction of cytosolic calcium ion concentration Sources: GOC:ai Subtypes: negative regulation of calcium ion transport into cytosol [GO:0010523], negative regulation of presynaptic cytosolic calcium concentration [GO:0099113] Definition: Any process that decreases the concentration of calcium ions in the cytosol.